choline biosynthetic process via phosphoryl-ethanolamine [GO:0033325] (biological process) Definition: The chemical reactions and pathways resulting in the formation of choline (2-hydroxyethyltrimethylammonium), via the intermediate phosphoryl-ethanolamine. Sources: GOC:mah, MetaCyc:PWY-3385 Also known as: choline anabolism via phosphoryl-ethanolamine, choline biosynthesis via phosphoryl-ethanolamine, choline formation via phosphoryl-ethanolamine, choline synthesis via phosphoryl-ethanolamine Relationships: is a type of GO:0042425